{
  "gene": "UniProtKB:Q92805",
  "gene_symbol": "GOLGA1",
  "term_label": "Unknown biological process",
  "gene_name": "Golgin subfamily A member 1",
  "term_id": "UNKNOWN:0002"
}